negative regulation of backward locomotion [GO:1905851] (biological process) Definition: Any process that stops, prevents or reduces the frequency, rate or extent of backward locomotion. Also known as: down regulation of backward locomotion, down-regulation of backward locomotion, downregulation of backward locomotion, inhibition of backward locomotion References: PMID:11717360 Sources: GOC:TermGenie, GO_REF:0000058 Relationships: is a type of negative regulation of locomotion [GO:0040013]; is a type of GO:0043058; negatively regulates backward locomotion [GO:0043057]